alpha-beta T cell activation by superantigen [GO:0042722] (biological process) Sources: GOC:jl Relationships: is_a GO:0046631 Also known as: alpha-beta T lymphocyte activation by superantigen, alpha-beta T-cell activation by superantigen, alpha-beta T-lymphocyte activation by superantigen Definition: The change in morphology and behavior of alpha-beta T cells resulting from exposure to a superantigen, a microbial antigen with an extremely potent activating effect on T cells that bear a specific variable region.